{
  "term_label": "negative regulation of vascular endothelial growth factor receptor signaling pathway",
  "gene_name": "Multimerin-1",
  "gene": "UniProtKB:Q13201",
  "term_id": "GO:0030948",
  "gene_symbol": "MMRN1"
}